{
  "gene": "UniProtKB:Q9NP95",
  "term_id": "GO:0008543",
  "gene_name": "Fibroblast growth factor 20",
  "gene_symbol": "FGF20",
  "term_label": "fibroblast growth factor receptor signaling pathway"
}